{
  "term_label": "small GTPase binding",
  "gene_symbol": "PLEKHG1",
  "gene_name": "Pleckstrin homology domain-containing family G member 1",
  "gene": "UniProtKB:Q9ULL1",
  "term_id": "GO:0031267"
}